{
  "term_label": "RNA polymerase II transcription regulatory region sequence-specific DNA binding",
  "gene_symbol": "ZNF823",
  "gene_name": "Zinc finger protein 823",
  "gene": "UniProtKB:P16415",
  "term_id": "GO:0000977"
}